{
  "term_id": "GO:0030175",
  "gene_symbol": "MYO10",
  "gene_name": "Unconventional myosin-X",
  "gene": "UniProtKB:Q9HD67",
  "term_label": "filopodium"
}